{
  "gene_symbol": "SLC8A3",
  "term_id": "GO:0006874",
  "term_label": "intracellular calcium ion homeostasis",
  "gene": "UniProtKB:P57103",
  "gene_name": "Sodium_calcium exchanger 3"
}